telodendria [GO:0120208] (cellular component) Subtypes: cone telodendria [GO:0120209], rod telodendria [GO:0120210] Relationships: is a type of neuron projection [GO:0043005] References: PMID:11074451, PMID:11506430, PMID:14755521, PMID:1646866, PMID:20533354, PMID:29127712, PMID:451992, PMID:8390352 Sources: GOC:cvs, GOC:krc Definition: Telodendria are projections that originate from the axon pedicle and form gap junctions with other neurons.